{
  "term_id": "GO:0016805",
  "gene_symbol": "CNDP2",
  "term_label": "dipeptidase activity",
  "gene": "UniProtKB:Q96KP4",
  "gene_name": "Cytosolic non-specific dipeptidase"
}